{
  "gene_symbol": "PSMA2",
  "term_label": "proteasome-mediated ubiquitin-dependent protein catabolic process",
  "gene": "UniProtKB:P25787",
  "term_id": "GO:0043161",
  "gene_name": "Proteasome subunit alpha type-2"
}